{
  "gene_symbol": "NYAP1",
  "term_id": "GO:0048812",
  "term_label": "neuron projection morphogenesis",
  "gene": "UniProtKB:Q6ZVC0",
  "gene_name": "Neuronal tyrosine-phosphorylated phosphoinositide-3-kinase adapter 1"
}